L-lysine transmembrane transport from lysosomal lumen to cytosol [GO:1904916] (biological process) Also known as: transmembrane L-lysine transport from lysosomal lumen to cytosol Definition: The directed movement of L-lysine from the lysosomal lumen across the lysosomal membrane and into the cytosol. References: PMID:22822152 Sources: GOC:TermGenie, GOC:kmv, GO_REF:0000078 Relationships: is a type of L-lysine transmembrane export from vacuole [GO:0089707]; is a type of transmembrane transport from lysosomal lumen to cytosol [GO:0170063]